carboxylate reductase activity [GO:0047770] (molecular function) Definition: Catalysis of the reaction: an aldehyde + acceptor + H2O = a carboxylate + reduced acceptor. Sources: EC:1.2.99.6, MetaCyc:CARBOXYLATE-REDUCTASE-RXN Also known as: aldehyde:(acceptor) oxidoreductase activity, aldehyde:acceptor oxidoreductase activity, carboxylic acid reductase activity Relationships: is a type of oxidoreductase activity, acting on the aldehyde or oxo group of donors [GO:0016903]